{
  "term_id": "GO:0004713",
  "gene_symbol": "WEE1",
  "gene": "UniProtKB:P30291",
  "gene_name": "Wee1-like protein kinase",
  "term_label": "protein tyrosine kinase activity"
}